{
  "gene_name": "TP53-binding protein 1",
  "gene_symbol": "TP53BP1",
  "term_id": "GO:0000077",
  "term_label": "DNA damage checkpoint signaling",
  "gene": "UniProtKB:Q12888"
}